{
  "term_label": "integrin alpha4-beta7 complex",
  "term_id": "GO:0034669",
  "gene_symbol": "ITGA4",
  "gene_name": "Integrin alpha-4",
  "gene": "UniProtKB:P13612"
}